{
  "gene_name": "Zinc finger protein 318",
  "gene_symbol": "ZNF318",
  "term_id": "GO:0005654",
  "gene": "UniProtKB:Q5VUA4",
  "term_label": "nucleoplasm"
}